sulfate assimilation [GO:0000103] (biological process) Regulation: regulated by GO:1900058; positively regulated by positive regulation of sulfate assimilation [GO:1900059] Definition: The pathways by which inorganic sulfate is processed and incorporated into sulfated compounds. Subtypes: sulfate assimilation via adenylyl sulfate reduction [GO:0010134], sulfate assimilation, phosphoadenylyl sulfate reduction by phosphoadenylyl-sulfate reductase (thioredoxin) [GO:0019379], dissimilatory sulfate reduction [GO:0019420] Sources: GOC:jl Also known as: sulphate assimilation, sulfate assimilation, phosphoadenylyl sulfate reduction by an oxidoreductase, acting on sulfur group of donors, NAD or NADP as acceptor, sulphate assimilation, phosphoadenylyl sulphate reduction by an oxidoreductase, acting on sulphur group of donors, NAD or NADP as acceptor Relationships: is a type of sulfur compound metabolic process [GO:0006790]